{
  "gene_symbol": "ZFP2",
  "gene": "UniProtKB:Q6ZN57",
  "gene_name": "Zinc finger protein ZFP2",
  "term_label": "RNA polymerase II cis-regulatory region sequence-specific DNA binding",
  "term_id": "GO:0000978"
}